{
  "gene": "UniProtKB:P49915",
  "term_label": "GMP synthase activity",
  "term_id": "GO:0003921",
  "gene_symbol": "GMPS",
  "gene_name": "GMP synthase [glutamine-hydrolyzing]"
}